root regeneration [GO:0062211] (biological process) Definition: The the regeneration process by which a damaged or lost root regrows or re-differentiates. This process may occur via de-differentiation and subsequent reprogramming of somatic cells or activation of existing undifferentiated (meristematic) cells to form a new root meristem and subsequently new root. References: PMID:27143753 Relationships: is a type of regeneration [GO:0031099]; is a type of root development [GO:0048364]